{
  "gene_symbol": "SLC39A6",
  "gene_name": "Zinc transporter ZIP6",
  "term_label": "intracellular monoatomic cation homeostasis",
  "term_id": "GO:0030003",
  "gene": "UniProtKB:Q13433"
}